sesquiterpene catabolic process [GO:0051763] (BP) Relationships: is_a terpene catabolic process [GO:0046247]; is a type of sesquiterpene metabolic process [GO:0051761] Subtypes: cadinene catabolic process [GO:1901927], alpha-copaene catabolic process [GO:1901930], bicyclogermacrene catabolic process [GO:1901933], beta-caryophyllene catabolic process [GO:1901936], (-)-exo-alpha-bergamotene catabolic process [GO:1901939] Definition: The chemical reactions and pathways resulting in the breakdown of sesquiterpenes, any of a class of terpenes of the formula C15H24 or a derivative of such a terpene. Sources: GOC:ai